toll-like receptor 13 signaling pathway [GO:0034178] (biological process) Definition: The series of molecular signals initiated by a ligand binding to the endolysosomal toll-like receptor 13. References: PMID:16551253, PMID:17328678 Sources: GOC:add Also known as: TLR13 signaling pathway, toll-like receptor 13 signalling pathway Relationships: is a type of endolysosomal toll-like receptor signaling pathway [GO:0140894] Regulation: regulated by GO:0034179; negatively regulated by negative regulation of toll-like receptor 13 signaling pathway [GO:0034180]; RO_0002213 by positive regulation of toll-like receptor 13 signaling pathway [GO:0034181]